{
  "gene_name": "Large ribosomal subunit protein mL51",
  "term_id": "GO:0005762",
  "term_label": "mitochondrial large ribosomal subunit",
  "gene_symbol": "MRPL51",
  "gene": "UniProtKB:Q4U2R6"
}